2,3-dihydroxy-p-cumate dioxygenase activity [GO:0018571] (MF) Also known as: 2,3-dihydroxy-p-cumate 3,4-dioxygenase, 2,3-dihydroxy-p-cumate-3,4-dioxygenase Definition: Catalysis of the reaction: 2,3-dihydroxy-p-cumate + O2 = 2-hydroxy-3-carboxy-6-oxo-7-methylocta-2,4-dienoate. Sources: RHEA:42568 Relationships: is a type of oxidoreductase activity, acting on single donors with incorporation of molecular oxygen, incorporation of two atoms of oxygen [GO:0016702]